response to prostaglandin D [GO:0071798] (biological process) Relationships: is a type of response to prostaglandin [GO:0034694]; is a type of response to alcohol [GO:0097305]; is a type of response to ketone [GO:1901654] Subtypes: cellular response to prostaglandin D stimulus [GO:0071799] Sources: GOC:sl Also known as: response to prostaglandin D stimulus Definition: Any process that results in a change in state or activity of a cell or an organism (in terms of movement, secretion, enzyme production, gene expression, etc.) as a result of a prostagladin D stimulus.